resolvin biosynthetic process [GO:0106295] (biological process) Definition: The chemical reactions and pathways resulting in the formation of resolvins, di- or trihydroxy fatty acids derived from omega-3 polyunsaturated fatty acids, specifically icosapentaenoic acid, docosahexaenoic acid and docosapentaenoic acid. References: PMID:24899309 Note: Resolvin biosynthesis is a combination of oxidation, reduction and hydrolysis reactions involving lipoxygenases and cyclooxygenases. Relationships: is a type of long-chain fatty acid biosynthetic process [GO:0042759]; is_a GO:0046173 Subtypes: D-series resolvin biosynthetic process [GO:0106296], E-series resolvin biosynthetic process [GO:0106297], 13-series resolvin biosynthetic process [GO:0106298]